{
  "gene_symbol": "SPART-AS1",
  "gene": "UniProtKB:P0CW21",
  "term_id": "UNKNOWN:0003",
  "term_label": "Unknown cellular component",
  "gene_name": "Putative uncharacterized protein SPART-AS1"
}